{
  "term_label": "chromatin DNA binding",
  "gene_symbol": "POLE3",
  "gene_name": "DNA polymerase epsilon subunit 3",
  "gene": "UniProtKB:Q9NRF9",
  "term_id": "GO:0031490"
}